{
  "term_label": "immunoglobulin mediated immune response",
  "gene_symbol": "IGHV4-28",
  "gene": "UniProtKB:A0A0C4DH34",
  "gene_name": "Immunoglobulin heavy variable 4-28",
  "term_id": "GO:0016064"
}